{
  "gene_symbol": "RREB1",
  "gene": "UniProtKB:Q92766",
  "term_id": "GO:0005634",
  "term_label": "nucleus",
  "gene_name": "Ras-responsive element-binding protein 1"
}